{
  "gene": "UniProtKB:P57088",
  "term_id": "GO:0061024",
  "term_label": "membrane organization",
  "gene_name": "Transmembrane protein 33",
  "gene_symbol": "TMEM33"
}